{
  "term_label": "nucleus",
  "term_id": "GO:0005634",
  "gene_name": "Jupiter microtubule associated homolog 1",
  "gene_symbol": "JPT1",
  "gene": "UniProtKB:Q9UK76"
}